negative regulation of branching involved in lung morphogenesis [GO:0061048] (biological process) Subtypes: negative regulation of bud outgrowth involved in lung branching [GO:0061112] Definition: Any process that decreases the rate, frequency, or extent of the process in which a highly ordered sequence of patterning events generates the branched structures of the lung, consisting of reiterated combinations of bud outgrowth, elongation, and dichotomous subdivision of terminal units. Sources: GOC:dph, GOC:yaf Relationships: is a type of negative regulation of multicellular organismal process [GO:0051241]; is a type of regulation of branching involved in lung morphogenesis [GO:0061046]; is a type of negative regulation of morphogenesis of an epithelium [GO:1905331]; negatively regulates epithelial tube branching involved in lung morphogenesis [GO:0060441]